{
  "term_id": "GO:0002286",
  "gene_name": "Interferon omega-1",
  "term_label": "T cell activation involved in immune response",
  "gene": "UniProtKB:P05000",
  "gene_symbol": "IFNW1"
}